{
  "term_label": "cAMP-dependent protein kinase complex",
  "gene_symbol": "PRKAR2B",
  "gene_name": "cAMP-dependent protein kinase type II-beta regulatory subunit",
  "term_id": "GO:0005952",
  "gene": "UniProtKB:P31323"
}